{
  "term_label": "intracellular signal transduction",
  "term_id": "GO:0035556",
  "gene": "UniProtKB:Q8TD08",
  "gene_name": "Mitogen-activated protein kinase 15",
  "gene_symbol": "MAPK15"
}